{
  "term_id": "GO:0141106",
  "term_label": "tRNA methyltransferase activator activity",
  "gene": "UniProtKB:Q9UI30",
  "gene_name": "Multifunctional methyltransferase subunit TRM112-like protein",
  "gene_symbol": "TRMT112"
}